{
  "term_label": "external side of plasma membrane",
  "term_id": "GO:0009897",
  "gene": "UniProtKB:Q9UP52",
  "gene_name": "Transferrin receptor protein 2",
  "gene_symbol": "TFR2"
}